free ubiquitin chain polymerization [GO:0010994] (biological process) Regulation: regulated by regulation of free ubiquitin chain polymerization [GO:1904542]; RO_0002212 by negative regulation of free ubiquitin chain polymerization [GO:1904543]; RO_0002213 by positive regulation of free ubiquitin chain polymerization [GO:1904544] Definition: The process of creating free ubiquitin chains, compounds composed of a large number of ubiquitin monomers. These chains are not conjugated to a protein. Relationships: is a type of GO:0051258; is part of ubiquitin recycling [GO:0010992] Sources: GOC:BHF, GOC:dph, GOC:tb